{
  "gene": "UniProtKB:P0C2L3",
  "gene_symbol": "FAM163B",
  "term_label": "Unknown cellular component",
  "term_id": "UNKNOWN:0003",
  "gene_name": "Protein FAM163B"
}